{
  "gene_symbol": "RHOBTB3",
  "gene": "UniProtKB:O94955",
  "gene_name": "Rho-related BTB domain-containing protein 3",
  "term_id": "GO:0043161",
  "term_label": "proteasome-mediated ubiquitin-dependent protein catabolic process"
}